{
  "term_label": "cell surface",
  "gene_symbol": "SCUBE1",
  "term_id": "GO:0009986",
  "gene": "UniProtKB:Q8IWY4",
  "gene_name": "Signal peptide, CUB and EGF-like domain-containing protein 1"
}